{
  "term_label": "cytosol",
  "gene": "UniProtKB:P45974",
  "gene_name": "Ubiquitin carboxyl-terminal hydrolase 5",
  "gene_symbol": "USP5",
  "term_id": "GO:0005829"
}